{
  "term_label": "protein kinase binding",
  "gene": "UniProtKB:Q8NFP9",
  "gene_symbol": "NBEA",
  "gene_name": "Neurobeachin",
  "term_id": "GO:0019901"
}